{
  "gene_name": "Phospholipase DDHD1",
  "term_label": "Unknown biological process",
  "gene_symbol": "DDHD1",
  "gene": "UniProtKB:Q8NEL9",
  "term_id": "UNKNOWN:0002"
}